{
  "gene_symbol": "IARS1",
  "term_label": "isoleucyl-tRNA aminoacylation",
  "gene_name": "Isoleucine--tRNA ligase, cytoplasmic",
  "term_id": "GO:0006428",
  "gene": "UniProtKB:P41252"
}